{
  "gene_symbol": "MLXIP",
  "term_label": "regulation of transcription by RNA polymerase II",
  "term_id": "GO:0006357",
  "gene": "UniProtKB:Q9HAP2",
  "gene_name": "MLX-interacting protein"
}